{
  "term_label": "serine-type endopeptidase inhibitor activity",
  "term_id": "GO:0004867",
  "gene_symbol": "SERPINA9",
  "gene": "UniProtKB:Q86WD7",
  "gene_name": "Serpin A9"
}